negative regulation of estrone secretion [GO:2000868] (BP) Relationships: is a type of negative regulation of steroid hormone secretion [GO:2000832]; is a type of regulation of estrone secretion [GO:2000867]; negatively regulates GO:0035943 Sources: GOC:sl Also known as: negative regulation of 3-hydroxy-1,3,5(10)-estratrien-17-one secretion, negative regulation of folliculin secretion Definition: Any process that stops, prevents or reduces the frequency, rate or extent of estrone secretion.